{
  "gene_symbol": "NATD1",
  "term_id": "UNKNOWN:0001",
  "gene": "UniProtKB:Q8N6N6",
  "term_label": "Unknown molecular function",
  "gene_name": "Protein NATD1"
}